{
  "gene_name": "Vimentin-type intermediate filament-associated coiled-coil protein",
  "term_label": "type III intermediate filament",
  "gene_symbol": "VMAC",
  "term_id": "GO:0045098",
  "gene": "UniProtKB:Q2NL98"
}